negative regulation of skeletal muscle hypertrophy [GO:1904205] (biological process) Definition: Any process that stops, prevents or reduces the frequency, rate or extent of skeletal muscle hypertrophy. References: PMID:23470307 Sources: GOC:TermGenie, GO_REF:0000058 Also known as: down regulation of skeletal muscle hypertrophy, down-regulation of skeletal muscle hypertrophy, downregulation of skeletal muscle hypertrophy, inhibition of skeletal muscle hypertrophy Relationships: is a type of negative regulation of muscle hypertrophy [GO:0014741]; is a type of negative regulation of muscle adaptation [GO:0014745]; is a type of regulation of skeletal muscle hypertrophy [GO:1904204]; negatively regulates skeletal muscle hypertrophy [GO:0014734]